{
  "term_id": "UNKNOWN:0002",
  "term_label": "Unknown biological process",
  "gene_name": "DPY30 domain-containing protein 2",
  "gene": "UniProtKB:Q96IM9",
  "gene_symbol": "DYDC2"
}